2-(acetamidomethylene)succinate hydrolase activity [GO:0047411] (molecular function) Definition: Catalysis of the reaction: 2 H2O + 2-(acetamidomethylene)succinate = CO2 + NH3 + succinate semialdehyde + acetate. Sources: EC:3.5.1.29, MetaCyc:3.5.1.29-RXN Also known as: 2-(acetamidomethylene)succinate amidohydrolase (deaminating, decarboxylating), alpha-(N-acetylaminomethylene)succinic acid hydrolase activity Relationships: is a type of hydrolase activity, acting on carbon-nitrogen (but not peptide) bonds, in linear amides [GO:0016811]